negative regulation of secondary cell wall biogenesis [GO:1901347] (biological process) Also known as: down regulation of secondary cell wall anabolism, down regulation of secondary cell wall biosynthetic process, down regulation of secondary cell wall formation, down regulation of secondary cell wall synthesis, down-regulation of secondary cell wall anabolism, down-regulation of secondary cell wall biosynthetic process, down-regulation of secondary cell wall formation, down-regulation of secondary cell wall synthesis, downregulation of secondary cell wall anabolism, downregulation of secondary cell wall biosynthetic process, downregulation of secondary cell wall formation, downregulation of secondary cell wall synthesis, inhibition of secondary cell wall anabolism, inhibition of secondary cell wall biosynthetic process, inhibition of secondary cell wall formation, inhibition of secondary cell wall synthesis, negative regulation of secondary cell wall anabolism, negative regulation of secondary cell wall biosynthetic process, negative regulation of secondary cell wall formation, negative regulation of secondary cell wall synthesis, down regulation of cellulose and pectin-containing secondary cell wall biogenesis, down regulation of plant-type secondary cell wall biogenesis, down regulation of secondary cell wall biogenesis, down-regulation of cellulose and pectin-containing secondary cell wall biogenesis, down-regulation of plant-type secondary cell wall biogenesis, down-regulation of secondary cell wall biogenesis, downregulation of cellulose and pectin-containing secondary cell wall biogenesis, downregulation of plant-type secondary cell wall biogenesis, downregulation of secondary cell wall biogenesis, inhibition of cellulose and pectin-containing secondary cell wall biogenesis, inhibition of plant-type secondary cell wall biogenesis, negative regulation of cellulose and pectin-containing secondary cell wall biogenesis, negative regulation of plant-type secondary cell wall biogenesis, inhibition of secondary cell wall biogenesis Relationships: is a type of negative regulation of cell wall organization or biogenesis [GO:1903339]; is a type of regulation of secondary cell wall biogenesis [GO:2000652]; negatively regulates plant-type secondary cell wall biogenesis [GO:0009834] Definition: Any process that stops, prevents or reduces the frequency, rate or extent of secondary cell wall biogenesis. Sources: GOC:TermGenie